{
  "term_id": "GO:0016020",
  "term_label": "membrane",
  "gene": "UniProtKB:Q68DH5",
  "gene_symbol": "LMBRD2",
  "gene_name": "G-protein coupled receptor-associated protein LMBRD2"
}